regulation of cholesterol import [GO:0060620] (biological process) Definition: Any process that modulates the rate, frequency or extent of cholesterol import. Cholesterol import is the directed movement of cholesterol into a cell or organelle. Subtypes: negative regulation of cholesterol import [GO:0060621], positive regulation of cholesterol import [GO:1904109] Relationships: is a type of regulation of cholesterol transport [GO:0032374]; regulates GO:0070508 Sources: GOC:BHF, GOC:dph, GOC:tb